{
  "term_label": "Unknown molecular function",
  "gene_symbol": "CLUHP3",
  "gene_name": "Putative protein CLUHP3",
  "gene": "UniProtKB:Q96NS8",
  "term_id": "UNKNOWN:0001"
}